regulation of TOR signaling [GO:0032006] (biological process) Definition: Any process that modulates the frequency, rate or extent of TOR signaling. Relationships: is a type of regulation of intracellular signal transduction [GO:1902531]; regulates GO:0031929 Sources: GOC:mah Also known as: regulation of TOR signaling pathway, regulation of TOR signalling pathway, regulation of target of rapamycin signaling pathway, regulation of target of rapamycin signalling pathway, regulation of TOR signaling cascade Subtypes: negative regulation of TOR signaling [GO:0032007], positive regulation of TOR signaling [GO:0032008], regulation of TORC1 signaling [GO:1903432], GO:1903939